{
  "gene_symbol": "CXorf1",
  "gene": "UniProtKB:O96002",
  "term_label": "Unknown molecular function",
  "gene_name": "Putative transmembrane protein CXorf1",
  "term_id": "UNKNOWN:0001"
}